{
  "gene": "UniProtKB:Q96HY7",
  "term_id": "UNKNOWN:0001",
  "gene_name": "2-oxoadipate dehydrogenase complex component E1",
  "gene_symbol": "DHTKD1",
  "term_label": "Unknown molecular function"
}